{
  "term_id": "GO:0005025",
  "term_label": "transforming growth factor beta receptor activity, type I",
  "gene_name": "Bone morphogenetic protein receptor type-1B",
  "gene": "UniProtKB:O00238",
  "gene_symbol": "BMPR1B"
}